{
  "gene_symbol": "OR10T2",
  "gene_name": "Olfactory receptor 10T2",
  "term_id": "GO:0016020",
  "gene": "UniProtKB:Q8NGX3",
  "term_label": "membrane"
}